{
  "gene_symbol": "DES",
  "gene_name": "Desmin",
  "term_id": "GO:0060538",
  "term_label": "skeletal muscle organ development",
  "gene": "UniProtKB:P17661"
}